positive regulation of triglyceride lipase activity [GO:0061365] (biological process) Also known as: positive regulation of TAG activity Subtypes: GO:0051006 Relationships: is a type of positive regulation of lipase activity [GO:0060193]; positively regulates triacylglycerol lipase activity [GO:0004806] Definition: Any process that increases the activity of triglyceride lipase. Sources: GOC:dph